{
  "gene": "UniProtKB:P14550",
  "gene_symbol": "AKR1A1",
  "term_id": "GO:0004032",
  "gene_name": "Aldo-keto reductase family 1 member A1",
  "term_label": "aldose reductase (NADPH) activity"
}